{
  "gene": "UniProtKB:Q8IZA0",
  "gene_symbol": "KIAA0319L",
  "term_label": "neuron migration",
  "term_id": "GO:0001764",
  "gene_name": "Dyslexia-associated protein KIAA0319-like protein"
}